indole biosynthetic process [GO:0042432] (biological process) Also known as: indole anabolism, indole biosynthesis, indole formation, indole synthesis Definition: The chemical reactions and pathways resulting in the formation of indole (2,3-benzopyrrole), the basis of many biologically active substances (e.g. serotonin, tryptophan). Sources: GOC:jl Relationships: is_a indole metabolic process [GO:0042431]; is a type of GO:0042435